{
  "gene_symbol": "DSE",
  "term_id": "UNKNOWN:0003",
  "gene_name": "Dermatan-sulfate epimerase",
  "gene": "UniProtKB:Q9UL01",
  "term_label": "Unknown cellular component"
}